{
  "term_label": "neutrophil chemotaxis",
  "gene_symbol": "TREM1",
  "term_id": "GO:0030593",
  "gene_name": "Triggering receptor expressed on myeloid cells 1",
  "gene": "UniProtKB:Q9NP99"
}